{
  "gene_symbol": "ATR",
  "term_label": "nucleus",
  "gene": "UniProtKB:Q13535",
  "gene_name": "Serine_threonine-protein kinase ATR",
  "term_id": "GO:0005634"
}